mitochondrial thiamine pyrophosphate transmembrane transport [GO:1990545] (BP) Definition: The process in which thiamine pyrophosphate is transported across a mitochondrial membrane, into or out of the mitochondrion. References: PMID:12411483 Relationships: is a type of thiamine pyrophosphate transmembrane transport [GO:0030974]